flavonol-3-O-glucoside glucosyltransferase activity [GO:0033838] (molecular function) Relationships: is a type of glucosyltransferase activity [GO:0046527] Also known as: UDP-glucose:flavonol-3-O-glucoside 2''-O-beta-D-glucosyltransferase activity Sources: EC:2.4.1.239 Definition: Catalysis of the reaction: UDP-glucose + a flavonol 3-O-beta-D-glucoside = UDP + a flavonol 3-O-beta-D-glucosyl-(1->2)-beta-D-glucoside.